{
  "gene_name": "Serine_threonine-protein kinase PLK4",
  "term_label": "Unknown biological process",
  "gene_symbol": "PLK4",
  "term_id": "UNKNOWN:0002",
  "gene": "UniProtKB:O00444"
}